{
  "term_label": "Unknown biological process",
  "term_id": "UNKNOWN:0002",
  "gene_symbol": "PCBD2",
  "gene": "UniProtKB:Q9H0N5",
  "gene_name": "Pterin-4-alpha-carbinolamine dehydratase 2"
}